{
  "gene_symbol": "CDH26",
  "gene": "UniProtKB:Q8IXH8",
  "term_label": "cadherin binding",
  "term_id": "GO:0045296",
  "gene_name": "Cadherin-like protein 26"
}